{
  "term_id": "GO:0005886",
  "gene": "UniProtKB:Q9H190",
  "term_label": "plasma membrane",
  "gene_name": "Syntenin-2",
  "gene_symbol": "SDCBP2"
}